{
  "term_label": "regulation of transcription by RNA polymerase II",
  "gene": "UniProtKB:Q6NX49",
  "gene_name": "Zinc finger protein 544",
  "gene_symbol": "ZNF544",
  "term_id": "GO:0006357"
}